{
  "gene_name": "Olfactory receptor 7A5",
  "term_id": "GO:0005886",
  "gene_symbol": "OR7A5",
  "gene": "UniProtKB:Q15622",
  "term_label": "plasma membrane"
}